biomineral tissue development [GO:0031214] (biological process) Definition: Formation of hard tissues that consist mainly of inorganic compounds, and also contain a small amounts of organic matrices that are believed to play important roles in their formation. Regulation: regulated by GO:0070167; negatively regulated by negative regulation of biomineral tissue development [GO:0070168]; positively regulated by positive regulation of biomineral tissue development [GO:0070169] References: PMID:15132736 Subtypes: GO:0030282, shell calcification [GO:0031215], tooth mineralization [GO:0034505], chitin-based cuticle sclerotization by biomineralization [GO:0036340], GO:0045299 Relationships: is a type of tissue development [GO:0009888]; is part of GO:0048513